dynein heavy chain binding [GO:0045504] (molecular function) Definition: Binding to a heavy chain of the dynein complex. Sources: GOC:bf Relationships: is a type of protein binding [GO:0005515]